{
  "term_label": "Unknown biological process",
  "gene": "UniProtKB:Q13442",
  "gene_name": "28 kDa heat- and acid-stable phosphoprotein",
  "term_id": "UNKNOWN:0002",
  "gene_symbol": "PDAP1"
}